{
  "gene": "UniProtKB:P02808",
  "gene_symbol": "STATH",
  "term_id": "GO:0061844",
  "gene_name": "Statherin",
  "term_label": "antimicrobial humoral immune response mediated by antimicrobial peptide"
}